{
  "gene_symbol": "C21orf58",
  "term_label": "Unknown biological process",
  "gene": "UniProtKB:P58505",
  "term_id": "UNKNOWN:0002",
  "gene_name": "Uncharacterized protein C21orf58"
}